{
  "gene": "UniProtKB:H3BQB6",
  "term_label": "tubulin binding",
  "gene_name": "Stathmin domain-containing protein 1",
  "term_id": "GO:0015631",
  "gene_symbol": "STMND1"
}